{
  "term_id": "GO:0031681",
  "gene": "UniProtKB:P59768",
  "term_label": "G-protein beta-subunit binding",
  "gene_symbol": "GNG2",
  "gene_name": "Guanine nucleotide-binding protein G(I)_G(S)_G(O) subunit gamma-2"
}